{
  "term_id": "GO:0000978",
  "gene_symbol": "PROX1",
  "gene_name": "Prospero homeobox protein 1",
  "term_label": "RNA polymerase II cis-regulatory region sequence-specific DNA binding",
  "gene": "UniProtKB:Q92786"
}